{
  "term_label": "negative regulation of canonical NF-kappaB signal transduction",
  "gene": "UniProtKB:P25963",
  "term_id": "GO:0043124",
  "gene_name": "NF-kappa-B inhibitor alpha",
  "gene_symbol": "NFKBIA"
}